{
  "gene_symbol": "MT-ND1",
  "gene_name": "NADH-ubiquinone oxidoreductase chain 1",
  "term_label": "respiratory chain complex I",
  "gene": "UniProtKB:P03886",
  "term_id": "GO:0045271"
}